(+)-thujopsene synthase activity [GO:0102879] (molecular function) Definition: Catalysis of the reaction: 2-trans,6-trans-farnesyl diphosphate = (+)-thujopsene + diphosphoric acid. Relationships: is a type of GO:0016838 Sources: GOC:pz, RHEA:30375